alpha7-beta1 integrin-laminin alpha-2 complex [GO:0071136] (CC) References: PMID:17598176 Definition: A protein complex that consists of an alpha7-beta1 integrin complex bound to laminin alpha-2. Also known as: ITGA7-ITGB1-LAMA2 complex Relationships: is a type of plasma membrane protein complex [GO:0098797]